{
  "term_label": "double-strand break repair via homologous recombination",
  "gene_symbol": "MCM9",
  "term_id": "GO:0000724",
  "gene_name": "DNA helicase MCM9",
  "gene": "UniProtKB:Q9NXL9"
}